galactarate biosynthetic process [GO:0046357] (biological process) Also known as: galactarate anabolism, galactarate biosynthesis, galactarate formation, galactarate synthesis, D-galactarate anabolism, D-galactarate biosynthesis, D-galactarate biosynthetic process, D-galactarate formation, D-galactarate synthesis Sources: GOC:pr, ISBN:0198506732 Definition: The chemical reactions and pathways resulting in the formation of galactarate, the anion of galactaric acid. Relationships: is_a GO:0019578; is a type of galactarate metabolic process [GO:0019580]